{
  "gene_symbol": "PRDM1",
  "term_label": "nucleus",
  "gene_name": "PR domain zinc finger protein 1",
  "gene": "UniProtKB:O75626",
  "term_id": "GO:0005634"
}